{
  "gene": "UniProtKB:Q96L33",
  "gene_symbol": "RHOV",
  "term_label": "GTPase activity",
  "term_id": "GO:0003924",
  "gene_name": "Rho-related GTP-binding protein RhoV"
}